{
  "gene_symbol": "STON1",
  "gene_name": "Stonin-1",
  "term_label": "synaptic vesicle",
  "gene": "UniProtKB:Q9Y6Q2",
  "term_id": "GO:0008021"
}